{
  "term_id": "GO:0009267",
  "gene_symbol": "ATG14",
  "gene_name": "Beclin 1-associated autophagy-related key regulator",
  "gene": "UniProtKB:Q6ZNE5",
  "term_label": "cellular response to starvation"
}